{
  "term_id": "GO:0004140",
  "gene_name": "Bifunctional coenzyme A synthase",
  "gene": "UniProtKB:Q13057",
  "gene_symbol": "COASY",
  "term_label": "dephospho-CoA kinase activity"
}